{
  "gene_symbol": "TCF7",
  "term_label": "DNA-binding transcription factor activity, RNA polymerase II-specific",
  "gene_name": "Transcription factor 7",
  "term_id": "GO:0000981",
  "gene": "UniProtKB:P36402"
}